lipid export from cell [GO:0140353] (BP) Definition: The directed movement of a lipid from a cell, into the extracellular region. Sources: GOC:pg Also known as: lipid efflux Relationships: is a type of lipid transport [GO:0006869]; is a type of GO:0140352 Subtypes: prostaglandin secretion [GO:0032310], steroid hormone secretion [GO:0035929], GO:0035936, GO:0035941, GO:0035942, juvenile hormone secretion [GO:0045443]